{
  "gene": "UniProtKB:Q5TA76",
  "term_id": "UNKNOWN:0001",
  "gene_symbol": "LCE3A",
  "term_label": "Unknown molecular function",
  "gene_name": "Late cornified envelope protein 3A"
}